tubulin folding cofactor complex [GO:1990727] (cellular component) Definition: A multimeric protein complex involved in tubulin alpha-beta-subunit folding assembly consisting of beta-tubulin-TFC-D, alpha-tubulin-TFC-E and TFC-C, through which tubulin subunit association and dimer release occur. References: PMID:12445400 Sources: GOC:vw Relationships: is a type of GO:0032991